protein secretion by the type IX secretion system [GO:0160303] (biological process) Also known as: Por secretion system, PorSS, T9SS References: PMID:19966289, PMID:37043368, PMID:40490843 Definition: The process by which proteins are transported from the periplasmic space across the outer membrane of Bacteroidota bacteria via the type IX secretion system (T9SS). Relationships: is a type of protein secretion [GO:0009306]; is a type of protein transmembrane transport [GO:0071806]